DNA-7-methylguanine glycosylase activity [GO:0043916] (molecular function) Relationships: is a type of alkylbase DNA N-glycosylase activity [GO:0003905] References: PMID:16468998 Sources: GOC:jl Definition: Catalysis of the reaction: DNA containing 7-methylguanine + H2O = DNA with abasic site + 7-methylguanine. This reaction is the hydrolysis of DNA by cleavage of the N-C1' glycosidic bond between the damaged DNA 7-methylguanine and the deoxyribose sugar to remove the 7-methylguanine, leaving an abasic site.